tissue homeostasis [GO:0001894] (biological process) Subtypes: retina homeostasis [GO:0001895], epithelial structure maintenance [GO:0010669], GO:0035633, maintenance of lens transparency [GO:0036438], bone resorption [GO:0045453], amnioserosa maintenance [GO:0046665], homeostasis of number of cells within a tissue [GO:0048873], compartment boundary maintenance [GO:0060289], inhibition of non-skeletal tissue mineralization [GO:0140928], GO:1990079 Sources: GOC:add, GOC:isa_complete Relationships: is a type of anatomical structure homeostasis [GO:0060249]; is part of multicellular organismal-level homeostasis [GO:0048871] Also known as: tissue maintenance Definition: A homeostatic process involved in the maintenance of an internal steady state within a defined tissue of an organism, including control of cellular proliferation and death and control of metabolic function.